{
  "gene_symbol": "ADAM9",
  "gene": "UniProtKB:Q13443",
  "gene_name": "Disintegrin and metalloproteinase domain-containing protein 9",
  "term_id": "GO:0005178",
  "term_label": "integrin binding"
}